{
  "gene": "UniProtKB:Q14766",
  "gene_symbol": "LTBP1",
  "term_id": "GO:0005615",
  "gene_name": "Latent-transforming growth factor beta-binding protein 1",
  "term_label": "extracellular space"
}